{
  "gene_name": "Small proline-rich protein 2D",
  "term_label": "Unknown molecular function",
  "term_id": "UNKNOWN:0001",
  "gene": "UniProtKB:P22532",
  "gene_symbol": "SPRR2D"
}